negative regulation of Rho guanyl-nucleotide exchange factor activity [GO:2001107] (biological process) Sources: GOC:obol Relationships: is a type of negative regulation of guanyl-nucleotide exchange factor activity [GO:1905098] Definition: Any process that stops, prevents or reduces the frequency, rate or extent of Rho guanyl-nucleotide exchange factor activity. Also known as: negative regulation of Rho guanine nucleotide exchange factor, negative regulation of RhoGEF